transcription elongation by RNA polymerase I [GO:0006362] (biological process) Sources: GOC:mah, GOC:txnOH Also known as: RNA elongation from Pol I promoter, transcription elongation from RNA polymerase I promoter, RNA polymerase I transcription elongation factor activity, transcription elongation from RNA polymerase I promoter for nuclear large rRNA transcript Regulation: regulated by regulation of transcription elongation by RNA polymerase I [GO:2001207]; negatively regulated by negative regulation of transcription elongation by RNA polymerase I [GO:2001208]; positively regulated by GO:2001209 Relationships: is a type of DNA-templated transcription elongation [GO:0006354]; is part of GO:0042790 Definition: The extension of an RNA molecule after transcription initiation and promoter clearance at an RNA polymerase I specific promoter by the addition of ribonucleotides catalyzed by RNA polymerase I.